neurotransmitter-gated ion channel clustering [GO:0072578] (biological process) References: PMID:20843816 Sources: GOC:dsf Subtypes: glycine receptor clustering [GO:0072579], GO:0097112, NMDA glutamate receptor clustering [GO:0097114], GO:0097688 Relationships: is a type of receptor clustering [GO:0043113]; is part of synapse organization [GO:0050808] Definition: The receptor clustering process in which neurotransmitter-gated ion channels are localized to distinct domains in the cell membrane.